{
  "gene_symbol": "CRY1",
  "gene_name": "Cryptochrome-1",
  "term_id": "GO:0032922",
  "gene": "UniProtKB:Q16526",
  "term_label": "circadian regulation of gene expression"
}